 [go#gocheck:do:not:annotate] Note: Term not to be used for direct annotation